positive regulation of mitochondrial depolarization [GO:0051901] (biological process) Sources: GOC:ai Relationships: is a type of regulation of mitochondrial depolarization [GO:0051900]; is a type of positive regulation of membrane depolarization [GO:1904181]; positively regulates mitochondrial depolarization [GO:0051882] Definition: Any process that activates, maintains or increases the frequency, rate or extent of the change in the membrane potential of the mitochondria from negative to positive. Also known as: up regulation of mitochondrial depolarization, up-regulation of mitochondrial depolarization, upregulation of mitochondrial depolarization, activation of mitochondrial depolarization, stimulation of mitochondrial depolarization